thiazole synthase complex [GO:1902507] (CC) Relationships: is a type of GO:1990228 Definition: A protein complex which is capable of thiazole synthase activity. References: PMID:12650933 Sources: GOC:TermGenie, GOC:bhm